regulation of bicellular tight junction assembly [GO:2000810] (biological process) Definition: Any process that modulates the frequency, rate or extent of tight junction assembly. Sources: GOC:BHF Also known as: regulation of tight junction formation Relationships: is a type of regulation of cell junction assembly [GO:1901888]; regulates GO:0070830 Subtypes: negative regulation of bicellular tight junction assembly [GO:1903347], positive regulation of bicellular tight junction assembly [GO:1903348]